methanol dehydrogenase (NAD+) activity [GO:0050093] (molecular function) Relationships: is a type of alcohol dehydrogenase (NAD+) activity [GO:0004022] Also known as: methanol dehydrogenase activity, methanol:NAD+ oxidoreductase activity Sources: EC:1.1.1.244, RHEA:19401 Definition: Catalysis of the reaction: methanol + NAD+ = formaldehyde + H+ + NADH.